{
  "gene": "UniProtKB:Q96LD1",
  "gene_symbol": "SGCZ",
  "gene_name": "Zeta-sarcoglycan",
  "term_id": "GO:0016012",
  "term_label": "sarcoglycan complex"
}